{
  "gene_symbol": "CASP1",
  "gene_name": "Caspase-1",
  "gene": "UniProtKB:P29466",
  "term_id": "GO:0097169",
  "term_label": "AIM2 inflammasome complex"
}